{
  "term_label": "Unknown biological process",
  "gene_name": "Protein-arginine deiminase type-3",
  "gene": "UniProtKB:Q9ULW8",
  "term_id": "UNKNOWN:0002",
  "gene_symbol": "PADI3"
}